{
  "term_label": "cell surface",
  "gene_name": "Leucine-rich repeat and fibronectin type-III domain-containing protein 5",
  "gene": "UniProtKB:Q96NI6",
  "term_id": "GO:0009986",
  "gene_symbol": "LRFN5"
}